RNA pseudouridylation guide activity [GO:0030558] (molecular function) Subtypes: rRNA pseudouridylation guide activity [GO:0030559], tRNA pseudouridylation guide activity [GO:0030560], snRNA pseudouridylation guide activity [GO:0030565] References: PMID:12457565 Sources: GOC:mah Note: Note that this term describes the activity of a nucleic acid, usually RNA, gene product that interacts with other RNA molecules via base pairing; it should not be used to annotate proteins. Definition: Specifies the site of pseudouridylation in an RNA molecule by base pairing with a short sequence around the target residue. Relationships: is_a RNA modification guide activity [GO:0030555]